angioblast cell differentiation [GO:0035779] (biological process) Definition: The process in which a relatively unspecialized cell acquires the specialized structural and/or functional features of an angioblast cell. Angioblasts are one of the two products formed from hemangioblast cells (the other being pluripotent hemopoietic stem cells). Sources: CL:0000566, GOC:yaf Also known as: angioblastic mesenchymal cell differentiation Relationships: is a type of GO:0048863; is part of blood vessel development [GO:0001568]